{
  "gene": "UniProtKB:Q9NPB6",
  "gene_symbol": "PARD6A",
  "term_id": "GO:0005938",
  "term_label": "cell cortex",
  "gene_name": "Partitioning defective 6 homolog alpha"
}